{
  "gene_name": "Acetylcholine receptor subunit delta",
  "term_id": "GO:0007268",
  "gene": "UniProtKB:Q07001",
  "gene_symbol": "CHRND",
  "term_label": "chemical synaptic transmission"
}